venom-mediated mast cell degranulation [GO:0044480] (biological process) References: PMID:21549739 Sources: GOC:fj, GOC:jl Relationships: is a type of venom-mediated perturbation of mast cell degranulation [GO:0044479] Definition: A process in which an organism initiates, promotes, or enhances mast cell degranulation in another organism via the action of a venom. Also known as: envenomation resulting in positive regulation of mast cell degranulation in another organism, envenomation resulting in positive regulation of mast cell degranulation in other organism